{
  "gene_name": "Arginase-2, mitochondrial",
  "term_id": "GO:0030145",
  "gene": "UniProtKB:P78540",
  "term_label": "manganese ion binding",
  "gene_symbol": "ARG2"
}